acrosomal vesicle [GO:0001669] (CC) Definition: A structure in the head of a spermatozoon that contains acid hydrolases, and is concerned with the breakdown of the outer membrane of the ovum during fertilization. It lies just beneath the plasma membrane and is derived from the lysosome. Sources: ISBN:0124325653, ISBN:0198506732 Also known as: acrosomal granule, acrosome Relationships: is a type of GO:0030141